base-excision repair [GO:0006284] (biological process) Definition: In base excision repair, an altered base is removed by a DNA glycosylase enzyme, followed by excision of the resulting sugar phosphate. The small gap left in the DNA helix is filled in by the sequential action of DNA polymerase and DNA ligase. Also known as: BER Sources: ISBN:0815316194 Subtypes: telomere maintenance via base-excision repair [GO:0097698] Relationships: is a type of DNA repair [GO:0006281] Regulation: regulated by GO:1905051; negatively regulated by GO:1905052; positively regulated by positive regulation of base-excision repair [GO:1905053]